{
  "gene_symbol": "CSHL1",
  "term_id": "GO:0005179",
  "gene_name": "Chorionic somatomammotropin hormone-like 1",
  "gene": "UniProtKB:Q14406",
  "term_label": "hormone activity"
}